{
  "gene": "UniProtKB:A8MX34",
  "gene_symbol": "KRTAP29-1",
  "term_id": "UNKNOWN:0003",
  "gene_name": "Keratin-associated protein 29-1",
  "term_label": "Unknown cellular component"
}